elaioplast organization [GO:0043579] (biological process) Relationships: is a type of GO:0009659 Definition: A process that is carried out at the cellular level which results in the assembly, arrangement of constituent parts, or disassembly of an elaioplast, a leucoplast in which oil is stored. Also known as: elaioplast organisation, elaioplast organization and biogenesis Sources: GOC:jl